{
  "gene_name": "Gamma-aminobutyric acid receptor subunit gamma-1",
  "term_label": "postsynapse",
  "gene_symbol": "GABRG1",
  "term_id": "GO:0098794",
  "gene": "UniProtKB:Q8N1C3"
}